positive regulation of vacuole organization [GO:0044090] (biological process) Sources: GOC:jl, GOC:mah Also known as: positive regulation of vacuole organisation, positive regulation of vacuole biogenesis Subtypes: positive regulation of vacuole fusion, non-autophagic [GO:0061191], GO:1905673, GO:2000786 Relationships: is a type of positive regulation of organelle organization [GO:0010638]; is a type of regulation of vacuole organization [GO:0044088]; positively regulates vacuole organization [GO:0007033] Definition: Any process that activates or increases the frequency, rate or extent of a process involved in the formation, arrangement of constituent parts, or disassembly of a vacuole.